carbon catabolite repression of transcription from RNA polymerase II promoter by glucose [GO:0000433] (biological process) Definition: A transcription regulation process in which the presence of glucose leads to a decrease in the frequency, rate, or extent of transcription of specific RNA polymerase II-transcribed genes involved in the metabolism of other carbon sources. Carbon catabolite repression is a mechanism of genetic regulation which the accumulation of catabolites of one substance in the cell represses the formation of enzymes that contribute to the catabolism of other substances. Relationships: is_a carbon catabolite repression of transcription by glucose [GO:0045014]; is a type of negative regulation of transcription from RNA polymerase II promoter by glucose [GO:0061987] Sources: GOC:krc Also known as: down regulation of transcription from RNA polymerase II promoter by glucose, down-regulation of transcription from RNA polymerase II promoter by glucose, downregulation of transcription from RNA polymerase II promoter by glucose, inhibition of transcription from RNA polymerase II promoter by glucose